natural killer cell activation [GO:0030101] (BP) Also known as: NK cell activation Sources: GOC:mgi_curators, ISBN:0781735149 Definition: The change in morphology and behavior of a natural killer cell in response to a cytokine, chemokine, cellular ligand, or soluble factor. Subtypes: natural killer cell differentiation [GO:0001779], natural killer cell proliferation [GO:0001787], natural killer cell activation involved in immune response [GO:0002323] Relationships: is a type of GO:0046649 Regulation: regulated by regulation of natural killer cell activation [GO:0032814]; negatively regulated by negative regulation of natural killer cell activation [GO:0032815]; positively regulated by positive regulation of natural killer cell activation [GO:0032816]